{
  "gene": "UniProtKB:Q96AE7",
  "term_id": "GO:0044782",
  "term_label": "cilium organization",
  "gene_symbol": "TTC17",
  "gene_name": "Tetratricopeptide repeat protein 17"
}